positive regulation of extracellular matrix constituent secretion [GO:0003331] (biological process) Sources: GOC:dph, GOC:tb Definition: Any process that increases the rate, frequency, or extent of the controlled release of molecules that form the extracellular matrix, including carbohydrates and glycoproteins by a cell or a group of cells. Relationships: is a type of GO:0003330; is a type of positive regulation of extracellular matrix organization [GO:1903055]; is a type of positive regulation of secretion by cell [GO:1903532]; positively regulates extracellular matrix constituent secretion [GO:0070278]